{
  "term_label": "plasma membrane",
  "gene": "UniProtKB:Q01959",
  "gene_symbol": "SLC6A3",
  "gene_name": "Sodium-dependent dopamine transporter",
  "term_id": "GO:0005886"
}